{
  "term_id": "GO:0004937",
  "gene_name": "Alpha-1B adrenergic receptor",
  "gene": "UniProtKB:P35368",
  "gene_symbol": "ADRA1B",
  "term_label": "alpha1-adrenergic receptor activity"
}